{
  "gene_name": "Adhesion G protein-coupled receptor B2",
  "term_id": "GO:0005886",
  "gene_symbol": "ADGRB2",
  "term_label": "plasma membrane",
  "gene": "UniProtKB:O60241"
}